{
  "gene_symbol": "IKBKE-AS1",
  "gene_name": "Putative uncharacterized protein IKBKE-AS1",
  "gene": "UniProtKB:Q96MC9",
  "term_id": "UNKNOWN:0003",
  "term_label": "Unknown cellular component"
}